response to interleukin-13 [GO:0035962] (biological process) Definition: Any process that results in a change in state or activity of a cell or an organism (in terms of movement, secretion, enzyme production, gene expression, etc.) as a result of an interleukin-13 stimulus. References: PMID:20100461 Sources: GOC:sjw Also known as: response to IL-13 Relationships: is a type of response to cytokine [GO:0034097] Subtypes: cellular response to interleukin-13 [GO:0035963]